{
  "gene": "UniProtKB:P34998",
  "term_label": "corticotropin-releasing hormone receptor activity",
  "gene_name": "Corticotropin-releasing factor receptor 1",
  "term_id": "GO:0043404",
  "gene_symbol": "CRHR1"
}